{
  "gene_symbol": "IFI16",
  "gene": "UniProtKB:Q16666",
  "gene_name": "Gamma-interferon-inducible protein 16",
  "term_id": "GO:0005829",
  "term_label": "cytosol"
}